{
  "gene_name": "Tyrosine-protein kinase Fgr",
  "gene_symbol": "FGR",
  "term_label": "cell differentiation",
  "term_id": "GO:0030154",
  "gene": "UniProtKB:P09769"
}